{
  "term_id": "GO:0005737",
  "gene_name": "Calcium_calmodulin-dependent protein kinase type II subunit alpha",
  "term_label": "cytoplasm",
  "gene": "UniProtKB:Q9UQM7",
  "gene_symbol": "CAMK2A"
}